opioid growth factor receptor signaling pathway [GO:0140626] (biological process) References: PMID:19675283, PMID:19923357 Definition: The series of molecular signals generated as a consequence of an opioid growth factor receptor binding to its physiological ligand, opioid growth factor (OGF, met-enkephalin). The OGF-OGFr complex leads to the increase in the synthesis of the selective cyclin-dependent kinase (CDK) inhibitor proteins, p12 (POLD4) and p16 (CDKN2A). Relationships: is a type of signal transduction [GO:0007165]; has part opioid growth factor receptor activity [GO:0140625] Note: Note that this term represents the activation of the zeta-opioid receptor. Do not confuse with GO:0038003 ; G protein-coupled opioid receptor signaling pathway, activated by the delta, kappa, mu, and nociceptin opioid receptors.